{
  "gene": "UniProtKB:Q86U70",
  "gene_symbol": "LDB1",
  "gene_name": "LIM domain-binding protein 1",
  "term_label": "nervous system development",
  "term_id": "GO:0007399"
}